{
  "term_id": "GO:0038187",
  "gene": "UniProtKB:Q6EIG7",
  "gene_symbol": "CLEC6A",
  "gene_name": "C-type lectin domain family 6 member A",
  "term_label": "pattern recognition receptor activity"
}